{
  "term_label": "structural constituent of synapse",
  "gene": "UniProtKB:O15020",
  "term_id": "GO:0098918",
  "gene_symbol": "SPTBN2",
  "gene_name": "Spectrin beta chain, non-erythrocytic 2"
}